{
  "term_id": "GO:0031265",
  "term_label": "CD95 death-inducing signaling complex",
  "gene": "UniProtKB:Q13158",
  "gene_name": "FAS-associated death domain protein",
  "gene_symbol": "FADD"
}